{
  "gene_symbol": "MRPS6",
  "term_label": "Unknown biological process",
  "gene_name": "Small ribosomal subunit protein bS6m",
  "gene": "UniProtKB:P82932",
  "term_id": "UNKNOWN:0002"
}